{
  "gene": "UniProtKB:Q56UN5",
  "term_id": "UNKNOWN:0001",
  "gene_name": "Mitogen-activated protein kinase kinase kinase 19",
  "term_label": "Unknown molecular function",
  "gene_symbol": "MAP3K19"
}